{
  "gene_symbol": "WDR38",
  "term_label": "Unknown cellular component",
  "term_id": "UNKNOWN:0003",
  "gene": "UniProtKB:Q5JTN6",
  "gene_name": "WD repeat-containing protein 38"
}